{
  "gene_symbol": "AGFG2",
  "gene_name": "Arf-GAP domain and FG repeat-containing protein 2",
  "term_label": "cytoplasmic vesicle",
  "gene": "UniProtKB:O95081",
  "term_id": "GO:0031410"
}